corticotropin-releasing hormone binding [GO:0051424] (MF) Relationships: is a type of peptide hormone binding [GO:0017046] References: PMID:7556876 Definition: Binding to corticotropin-releasing hormone, a polypeptide hormone involved in the stress response. It is released by the hypothalamus and stimulates the release of corticotropin by the anterior pituitary gland. Also known as: CRF binding, CRH binding, corticoliberin binding, corticotropin-releasing factor binding